{
  "gene_name": "HAUS augmin-like complex subunit 6",
  "term_label": "microtubule binding",
  "gene": "UniProtKB:Q7Z4H7",
  "term_id": "GO:0008017",
  "gene_symbol": "HAUS6"
}